negative regulation of astrocyte activation [GO:0061889] (BP) Relationships: is a type of GO:0048712; is a type of GO:0050866; is a type of GO:0061888; is a type of GO:0150079; negatively regulates GO:0048143 References: PMID:20005821 Sources: GOC:aruk, GOC:bc Definition: Any process that decreases the frequency, rate or extent of astrocyte activation.